{
  "term_id": "GO:0005634",
  "term_label": "nucleus",
  "gene": "UniProtKB:Q9UPV7",
  "gene_symbol": "PHF24",
  "gene_name": "PHD finger protein 24"
}